voltage-gated calcium channel activity [GO:0005245] (molecular function) Sources: GOC:mtg_transport, GOC:tb, ISBN:0815340729 Also known as: depolarization-activated calcium channel, depolarization-activated voltage gated calcium channel activity, depolarization-activated voltage-gated calcium channel, depolarization-activated voltage-gated calcium channel activity, voltage gated calcium channel activity, voltage-dependent calcium channel activity, voltage-gated calcium ion channel activity, voltage-sensitive calcium channel, dihydropyridine-sensitive calcium channel activity Regulation: regulated by regulation of voltage-gated calcium channel activity [GO:1901385]; negatively regulated by negative regulation of voltage-gated calcium channel activity [GO:1901386]; positively regulated by GO:1901387 Subtypes: GO:0008086, GO:0008331, low voltage-gated calcium channel activity [GO:0008332], voltage-gated calcium channel activity involved in cardiac muscle cell action potential [GO:0086007], voltage-gated calcium channel activity involved in regulation of cytosolic calcium levels [GO:0099511], voltage-gated calcium channel activity involved in positive regulation of presynaptic cytosolic calcium levels [GO:0099635], intermediate voltage-gated calcium channel activity [GO:1990028] Relationships: is_a GO:0005262; is a type of voltage-gated monoatomic cation channel activity [GO:0022843] Definition: Enables the transmembrane transfer of a calcium ion by a voltage-gated channel. A voltage-gated channel is a channel whose open state is dependent on the voltage across the membrane in which it is embedded.